iRhom2/ADAM17 sheddase complex [GO:0140910] (cellular component) Relationships: is a type of GO:0032991 Definition: A complex consisting of ADAM17 in complex with regulatory iRhoms and FERM domain containing proteins. References: PMID:29897336